{
  "gene": "UniProtKB:Q2M3X9",
  "term_label": "regulation of transcription by RNA polymerase II",
  "gene_symbol": "ZNF674",
  "term_id": "GO:0006357",
  "gene_name": "Zinc finger protein 674"
}